{
  "term_id": "GO:0006906",
  "gene_symbol": "STX6",
  "term_label": "vesicle fusion",
  "gene": "UniProtKB:O43752",
  "gene_name": "Syntaxin-6"
}